{
  "gene": "UniProtKB:Q8N5U6",
  "term_id": "GO:0061630",
  "term_label": "ubiquitin protein ligase activity",
  "gene_name": "E3 ubiquitin-protein ligase RNF10",
  "gene_symbol": "RNF10"
}